{
  "term_id": "UNKNOWN:0002",
  "term_label": "Unknown biological process",
  "gene_symbol": "PNN",
  "gene": "UniProtKB:Q9H307",
  "gene_name": "Pinin"
}